ureter epithelial cell differentiation [GO:0072192] (biological process) Definition: The process in which a relatively unspecialized cell acquires specialized features of an epithelial cell in the urothelium. The urothelium is the epithelial tube of the ureter. Sources: GOC:mtg_kidney_jan10 Relationships: is a type of epithelial cell differentiation [GO:0030855]; is part of GO:0072190